{
  "term_id": "UNKNOWN:0001",
  "gene_symbol": "NOL4L",
  "term_label": "Unknown molecular function",
  "gene": "UniProtKB:Q96MY1",
  "gene_name": "Nucleolar protein 4-like"
}